{
  "term_label": "deSUMOylase activity",
  "term_id": "GO:0016929",
  "gene_symbol": "SENP3",
  "gene_name": "Sentrin-specific protease 3",
  "gene": "UniProtKB:Q9H4L4"
}